{
  "term_label": "intracellular protein transport",
  "gene_symbol": "STX12",
  "gene": "UniProtKB:Q86Y82",
  "gene_name": "Syntaxin-12",
  "term_id": "GO:0006886"
}